positive regulation of neutrophil differentiation [GO:0045660] (BP) Definition: Any process that activates or increases the frequency, rate or extent of neutrophil differentiation. Also known as: up regulation of neutrophil differentiation, up-regulation of neutrophil differentiation, upregulation of neutrophil differentiation, activation of neutrophil differentiation, stimulation of neutrophil differentiation Sources: GOC:go_curators Relationships: is a type of GO:0030854; is a type of regulation of neutrophil differentiation [GO:0045658]; positively regulates neutrophil differentiation [GO:0030223]